Mo-molybdopterin cofactor catabolic process [GO:0032326] (biological process) Relationships: is a type of Mo-molybdopterin cofactor metabolic process [GO:0019720]; is a type of molybdopterin cofactor catabolic process [GO:0032325] Definition: The chemical reactions and pathways resulting in the breakdown of the Mo-molybdopterin cofactor, essential for the catalytic activity of some enzymes. The cofactor consists of a mononuclear molybdenum (Mo) ion coordinated by one or two molybdopterin ligands. Sources: GOC:mah Also known as: Moco catabolic process, Moco catabolism, Mo-molybdopterin cofactor breakdown, Mo-molybdopterin cofactor catabolism, Mo-molybdopterin cofactor degradation